all-trans-nonaprenyl-diphosphate synthase (geranyl-diphosphate specific) activity [GO:0052923] (molecular function) Definition: Catalysis of the reaction: 7 isopentenyl diphosphate + (2E)-geranyl diphosphate = all-trans-nonaprenyl diphosphate + 7 diphosphate. Sources: RHEA:27563 Also known as: SPP synthase activity, SPP-synthase activity, nonaprenyl diphosphate synthase activity, solPP synthase activity, solanesyl diphosphate synthetase activity, (E)-octaprenyl-diphosphate:isopentenyl-diphosphate octaprenyltranstransferase activity, all-trans-nonaprenyl-diphosphate synthase activity, nonaprenyl pyrophosphate synthetase activity, polyprenylpyrophosphate synthetase activity, solanesyl pyrophosphate synthetase activity, solanesyl-diphosphate synthase activity, terpenoidallyltransferase activity, terpenyl pyrophosphate synthetase activity, trans-octaprenyltranstransferase activity, trans-prenyltransferase activity Relationships: is_a GO:0120531